{
  "gene_name": "Uncharacterized protein",
  "gene": "UniProtKB:Q6YL49",
  "gene_symbol": "Q6YL49",
  "term_label": "Unknown molecular function",
  "term_id": "UNKNOWN:0001"
}